maintenance of polarity of embryonic epithelium [GO:0042250] (biological process) Definition: The maintenance of an established polarized embryonic epithelial sheet. Relationships: is_a establishment or maintenance of polarity of embryonic epithelium [GO:0016332] Sources: GOC:jl